MalFGK2 complex [GO:1990176] (cellular component) Also known as: MalF-MalG-MalK(2) complex, MalF-MalG-MalK-MalK complex, MalFGK(2) complex, maltose transport MalFGK2 complex, maltose transport complex, core subunit Note: The MalFGK2 complex lacks the maltose-binding subunit present in GO:1990060. Definition: Protein complex involved in maltose transport through the plasma membrane. In E. coli, the complex is a tetramer and consists of a cytoplasmic ATPase MalK homodimer together with a heterodimeric transmembrane subunit MalF-MalG. Relationships: is a type of GO:0098797; is part of GO:1990060 References: PMID:19250913 Sources: GOC:bhm